{
  "gene_symbol": "EPHA7",
  "gene": "UniProtKB:Q15375",
  "term_label": "plasma membrane",
  "term_id": "GO:0005886",
  "gene_name": "Ephrin type-A receptor 7"
}